chitin-based extracellular matrix [GO:0062129] (cellular component) References: PMID:23955854 Also known as: chitin-based ECM Relationships: is a type of specialized extracellular matrix [GO:0140047] Definition: Any constituent part of a chitin-based noncellular, hardened, or membranous extracellular matrix secreted from the apical surface of an epithelial sheet.